{
  "gene_name": "Metallothionein-1M",
  "term_id": "GO:0005737",
  "term_label": "cytoplasm",
  "gene_symbol": "MT1M",
  "gene": "UniProtKB:Q8N339"
}